{
  "term_label": "Unknown cellular component",
  "gene_symbol": "NPIPB12",
  "term_id": "UNKNOWN:0003",
  "gene": "UniProtKB:F8W0I5",
  "gene_name": "Nuclear pore complex-interacting protein family member B12"
}